{
  "gene_symbol": "STUB1",
  "gene": "UniProtKB:Q9UNE7",
  "gene_name": "E3 ubiquitin-protein ligase CHIP",
  "term_id": "GO:0006515",
  "term_label": "protein quality control for misfolded or incompletely synthesized proteins"
}